orexin secretion, neurotransmission [GO:0061585] (biological process) Definition: The controlled release of orexin from a cell in which orexin acts as a neurotransmitter. Also known as: hypocretin secretion, neurotransmission Relationships: is a type of peptide secretion, neurotransmission [GO:0061544]; is a type of orexin secretion [GO:0061584] Sources: GOC:dph